{
  "gene_symbol": "CALB2",
  "gene_name": "Calretinin",
  "term_id": "GO:0043195",
  "gene": "UniProtKB:P22676",
  "term_label": "terminal bouton"
}